{
  "gene_name": "Collagen triple helix repeat-containing protein 1",
  "term_id": "GO:0005737",
  "gene": "UniProtKB:Q96CG8",
  "gene_symbol": "CTHRC1",
  "term_label": "cytoplasm"
}